D-lactate-2-sulfatase activity [GO:0047825] (molecular function) Definition: Catalysis of the reaction: (R)-2-O-sulfolactate + H2O = (R)-lactate + H+ + sulfate. Sources: EC:3.1.6.17, RHEA:20337 Also known as: D-lactate-2-sulphatase activity, (S)-2-O-sulfolactate 2-sulfohydrolase activity Relationships: is a type of GO:0008484